{
  "term_id": "GO:0005085",
  "term_label": "guanyl-nucleotide exchange factor activity",
  "gene_symbol": "SOS2",
  "gene": "UniProtKB:Q07890",
  "gene_name": "Son of sevenless homolog 2"
}